N-retinylidene-phosphatidylethanolamine flippase activity [GO:0140347] (molecular function) References: PMID:10412977 Relationships: is_a glycerophospholipid flippase activity [GO:0140333] Also known as: N-retinylidene-phosphatidylethanolamine flippase activity (exoplasmic to cytosolic leaflet) Definition: Catalysis of the movement of N-retinylidene-N-retinylphosphatidylethanolamine from the exoplasmic to the cytosolic leaflet of a membrane, using energy from the hydrolysis of ATP.